{
  "gene_symbol": "NLRP9",
  "term_id": "UNKNOWN:0001",
  "gene": "UniProtKB:Q7RTR0",
  "term_label": "Unknown molecular function",
  "gene_name": "NACHT, LRR and PYD domains-containing protein 9"
}